positive regulation of cell-cell adhesion mediated by cadherin [GO:2000049] (biological process) Definition: Any process that activates or increases the frequency, rate or extent of cell-cell adhesion mediated by cadherin. Sources: GOC:obol Relationships: is a type of positive regulation of cell-cell adhesion [GO:0022409]; is a type of regulation of cell-cell adhesion mediated by cadherin [GO:2000047]; positively regulates cell-cell adhesion mediated by cadherin [GO:0044331]